phosphotransferase activity, nitrogenous group as acceptor [GO:0016775] (molecular function) Subtypes: arginine kinase activity [GO:0004054], GO:0004111, GO:0004673, phosphoenolpyruvate-protein phosphotransferase activity [GO:0008965], agmatine kinase activity [GO:0047633], ammonia kinase activity [GO:0047666], GO:0047715, GO:0047973, lombricine kinase activity [GO:0050059], opheline kinase activity [GO:0050154], taurocyamine kinase activity [GO:0050324] Definition: Catalysis of the transfer of a phosphorus-containing group from one compound (donor) to a nitrogenous group (acceptor). Sources: EC:2.7.3.- Relationships: is a type of GO:0016772